{
  "gene_symbol": "CREB3",
  "gene": "UniProtKB:O43889",
  "gene_name": "Cyclic AMP-responsive element-binding protein 3",
  "term_id": "GO:0006357",
  "term_label": "regulation of transcription by RNA polymerase II"
}